{
  "gene_name": "Hepatocyte growth factor receptor",
  "term_label": "receptor complex",
  "gene": "UniProtKB:P08581",
  "gene_symbol": "MET",
  "term_id": "GO:0043235"
}